{
  "gene_name": "Uncharacterized protein KIAA1614",
  "gene": "UniProtKB:Q5VZ46",
  "gene_symbol": "KIAA1614",
  "term_id": "GO:0016324",
  "term_label": "apical plasma membrane"
}